extrinsic component of endoplasmic reticulum membrane [GO:0042406] (cellular component) Sources: GOC:curators, GOC:dos Also known as: extrinsic to ER membrane, extrinsic to endoplasmic reticulum membrane Definition: The component of the endoplasmic reticulum membrane consisting of gene products and protein complexes that are loosely bound to one of its surfaces, but not integrated into the hydrophobic region. Relationships: is a type of GO:0031312; is part of endoplasmic reticulum membrane [GO:0005789]